{
  "gene_symbol": "TERT",
  "term_label": "telomerase RNA binding",
  "gene_name": "Telomerase reverse transcriptase",
  "gene": "UniProtKB:O14746",
  "term_id": "GO:0070034"
}